{
  "gene_name": "Voltage-dependent T-type calcium channel subunit alpha-1H",
  "term_id": "GO:0098703",
  "gene_symbol": "CACNA1H",
  "term_label": "calcium ion import across plasma membrane",
  "gene": "UniProtKB:O95180"
}